{
  "term_id": "GO:1904158",
  "gene_symbol": "SPAG17",
  "gene": "UniProtKB:Q6Q759",
  "term_label": "axonemal central apparatus assembly",
  "gene_name": "Sperm-associated antigen 17"
}